{
  "term_label": "DNA-binding transcription factor activity, RNA polymerase II-specific",
  "term_id": "GO:0000981",
  "gene": "UniProtKB:Q09FC8",
  "gene_name": "Zinc finger protein 415",
  "gene_symbol": "ZNF415"
}